acrylonitrile catabolic process [GO:0019256] (biological process) Relationships: is a type of GO:0042178; is a type of nitrile catabolic process [GO:0050899] References: PMID:1390687, PMID:3830164 Sources: GOC:ai Definition: The chemical reactions and pathways resulting in the breakdown of acrylonitrile, a colorless, volatile liquid with a pungent odor. Acrylonitrile is used in the production of acrylic fibers, plastics, and synthetic rubbers. Also known as: acrylonitrile breakdown, acrylonitrile catabolism, acrylonitrile degradation